{
  "gene": "UniProtKB:Q6ICL7",
  "term_label": "transmembrane transport",
  "term_id": "GO:0055085",
  "gene_symbol": "SLC35E4",
  "gene_name": "Solute carrier family 35 member E4"
}